{
  "gene_name": "E3 ubiquitin-protein ligase TRIM34",
  "gene": "UniProtKB:Q9BYJ4",
  "term_id": "GO:0010468",
  "gene_symbol": "TRIM34",
  "term_label": "regulation of gene expression"
}